{
  "term_id": "GO:0036393",
  "gene_name": "Lactoperoxidase",
  "term_label": "thiocyanate peroxidase activity",
  "gene_symbol": "LPO",
  "gene": "UniProtKB:P22079"
}